{
  "gene": "UniProtKB:O15078",
  "gene_name": "Centrosomal protein of 290 kDa",
  "term_label": "ciliary transition zone",
  "term_id": "GO:0035869",
  "gene_symbol": "CEP290"
}